{
  "gene_symbol": "TSG101",
  "gene": "UniProtKB:Q99816",
  "term_label": "endosome to lysosome transport",
  "term_id": "GO:0008333",
  "gene_name": "Tumor susceptibility gene 101 protein"
}